{
  "term_label": "neuron projection",
  "gene_symbol": "HTR3C",
  "gene": "UniProtKB:Q8WXA8",
  "gene_name": "5-hydroxytryptamine receptor 3C",
  "term_id": "GO:0043005"
}